BCOR complex [GO:0140261] (cellular component) Definition: A protein-containing complex that monoubiquitinates histone H2A on K119, thus it facilitates the maintenance of the transcriptionally repressive state of some genes, such as BCL6. It consists of the corepressor BCOR or BCORL1, a Polycomb group (PcG) and a SCF ubiquitin ligase subcomplexes. In mammals, the core subunits of the complex include the PcG and PcG-associated proteins NSPC1, RING1, RNF2, and RYBP and the components of the SCF ubiquitin ligase, SKP1, and FBXL10. References: PMID:16943429, PMID:22325352, PMID:24515802 Also known as: BCL6 corepressor (BCOR) complex, BCOR/BCORL1 complex, PRC1.1 complex, non-canonical BCOR-PRC1.1 complex, non-canonical PRC1-BCOR complex Relationships: is a type of nuclear ubiquitin ligase complex [GO:0000152]